{
  "gene_symbol": "MIEN1",
  "term_label": "negative regulation of apoptotic process",
  "gene_name": "Migration and invasion enhancer 1",
  "gene": "UniProtKB:Q9BRT3",
  "term_id": "GO:0043066"
}